{
  "gene_symbol": "FHL3",
  "term_id": "GO:0003712",
  "term_label": "transcription coregulator activity",
  "gene_name": "Four and a half LIM domains protein 3",
  "gene": "UniProtKB:Q13643"
}